{
  "term_id": "GO:0043153",
  "gene": "UniProtKB:P56645",
  "gene_name": "Period circadian protein homolog 3",
  "gene_symbol": "PER3",
  "term_label": "entrainment of circadian clock by photoperiod"
}